{
  "term_id": "GO:0045944",
  "gene": "UniProtKB:Q96NK8",
  "gene_name": "Neurogenic differentiation factor 6",
  "term_label": "positive regulation of transcription by RNA polymerase II",
  "gene_symbol": "NEUROD6"
}